{
  "term_label": "sodium ion transmembrane transport",
  "gene": "UniProtKB:Q99884",
  "gene_name": "Sodium-dependent proline transporter",
  "gene_symbol": "SLC6A7",
  "term_id": "GO:0035725"
}